{
  "term_id": "UNKNOWN:0002",
  "term_label": "Unknown biological process",
  "gene_name": "Renal cancer differentiation gene 1 protein",
  "gene": "UniProtKB:Q504U0",
  "gene_symbol": "C4orf46"
}